{
  "gene_symbol": "NEK2",
  "term_id": "GO:0007098",
  "term_label": "centrosome cycle",
  "gene_name": "Serine_threonine-protein kinase Nek2",
  "gene": "UniProtKB:P51955"
}